RNA splicing [GO:0008380] (biological process) Also known as: pre-mRNA splicing factor activity Regulation: negatively regulated by negative regulation of RNA splicing [GO:0033119]; positively regulated by positive regulation of RNA splicing [GO:0033120]; regulated by regulation of RNA splicing [GO:0043484] Subtypes: GO:0000375, RNA splicing, via endonucleolytic cleavage and ligation [GO:0000394], snoRNA splicing [GO:0034247] Definition: The process of removing sections of the primary RNA transcript to remove sequences not present in the mature form of the RNA and joining the remaining sections to form the mature form of the RNA. Sources: GOC:krc, GOC:mah Relationships: is a type of GO:0006396